{
  "gene_name": "ADP-ribosylation factor-like protein 11",
  "term_label": "vesicle-mediated transport",
  "gene": "UniProtKB:Q969Q4",
  "gene_symbol": "ARL11",
  "term_id": "GO:0016192"
}